detection of light stimulus [GO:0009583] (biological process) Subtypes: GO:0007602, detection of visible light [GO:0009584], detection of UV [GO:0009589], detection of light stimulus involved in sensory perception [GO:0050962] Sources: GOC:go_curators Relationships: is a type of response to light stimulus [GO:0009416]; is a type of detection of external stimulus [GO:0009581]; is a type of detection of abiotic stimulus [GO:0009582] Definition: The series of events in which a light stimulus (in the form of photons) is received and converted into a molecular signal. Also known as: detection of light, perception of light